{
  "gene": "UniProtKB:P28066",
  "gene_symbol": "PSMA5",
  "term_label": "nucleus",
  "term_id": "GO:0005634",
  "gene_name": "Proteasome subunit alpha type-5"
}